{
  "gene": "UniProtKB:Q9UBH0",
  "gene_symbol": "IL36RN",
  "gene_name": "Interleukin-36 receptor antagonist protein",
  "term_id": "GO:0006954",
  "term_label": "inflammatory response"
}